{
  "term_id": "GO:0097720",
  "gene_name": "Calmodulin-1",
  "gene": "UniProtKB:P0DP23",
  "term_label": "calcineurin-mediated signaling",
  "gene_symbol": "CALM1"
}